{
  "term_id": "GO:0048027",
  "gene": "UniProtKB:O60506",
  "gene_name": "Heterogeneous nuclear ribonucleoprotein Q",
  "gene_symbol": "SYNCRIP",
  "term_label": "mRNA 5'-UTR binding"
}